{
  "gene_symbol": "ITGA2B",
  "gene": "UniProtKB:P08514",
  "term_id": "GO:0038023",
  "term_label": "signaling receptor activity",
  "gene_name": "Integrin alpha-IIb"
}